HLA-A specific activating MHC class I receptor activity [GO:0030108] (molecular function) Relationships: is a type of activating MHC class I receptor activity [GO:0032397] Definition: Combining with a MHC class I molecule of the HLA-A subclass to mediate signaling that activates a lymphocyte. References: PMID:11929129, PMID:9368779 Sources: GOC:add, GOC:mah